positive regulation of sorocarp stalk cell differentiation [GO:0031287] (biological process) Definition: Any process that activates or increases the frequency, rate or extent of sorocarp stalk cell differentiation. An example of this process is found in Dictyostelium discoideum. Also known as: positive regulation of stalk cell differentiation, up regulation of stalk cell differentiation, up-regulation of stalk cell differentiation, upregulation of stalk cell differentiation, activation of stalk cell differentiation, stimulation of stalk cell differentiation References: PMID:4338436 Sources: GOC:kp, GOC:mtg_sensu Relationships: is a type of regulation of sorocarp stalk cell differentiation [GO:0031285]; is a type of positive regulation of response to nutrient levels [GO:0032109]; is a type of positive regulation of cell differentiation [GO:0045597]; is a type of GO:0075261; positively regulates GO:0031149